myosin heavy chain binding [GO:0032036] (molecular function) Definition: Binding to a heavy chain of a myosin complex. Sources: GOC:mah Relationships: is a type of myosin binding [GO:0017022] Subtypes: myosin head/neck binding [GO:0032028], myosin tail binding [GO:0032029], myosin I heavy chain binding [GO:0032037], GO:0032038, GO:0070854